{
  "gene_symbol": "TBC1D10B",
  "term_label": "GTPase activator activity",
  "term_id": "GO:0005096",
  "gene": "UniProtKB:Q4KMP7",
  "gene_name": "TBC1 domain family member 10B"
}